{
  "gene_symbol": "TINAG",
  "term_label": "extracellular space",
  "gene_name": "Tubulointerstitial nephritis antigen",
  "term_id": "GO:0005615",
  "gene": "UniProtKB:Q9UJW2"
}